{
  "gene_symbol": "ITGB4",
  "term_label": "cell-cell adhesion",
  "gene_name": "Integrin beta-4",
  "term_id": "GO:0098609",
  "gene": "UniProtKB:P16144"
}